{
  "term_label": "histone H3 acetyltransferase activity",
  "gene_name": "Histone acetyltransferase KAT6B",
  "term_id": "GO:0010484",
  "gene_symbol": "KAT6B",
  "gene": "UniProtKB:Q8WYB5"
}